{
  "gene_symbol": "DLL1",
  "gene_name": "Delta-like protein 1",
  "term_id": "GO:0005886",
  "gene": "UniProtKB:O00548",
  "term_label": "plasma membrane"
}